{
  "gene_name": "Complement component C6",
  "gene": "UniProtKB:P13671",
  "term_id": "GO:0006956",
  "term_label": "complement activation",
  "gene_symbol": "C6"
}